{
  "gene_symbol": "TRPC6",
  "term_label": "calcium ion transmembrane transport",
  "gene_name": "Short transient receptor potential channel 6",
  "gene": "UniProtKB:Q9Y210",
  "term_id": "GO:0070588"
}